infection cushion formation [GO:0075183] (biological process) Also known as: infection cushion formation on or near host Relationships: is a type of formation of infection structure [GO:0075015] Sources: GOC:pamgo_curators Definition: The process in which an organized mass of hyphae is formed and numerous infective hyphae develop from the hyphae mass. Regulation: regulated by regulation of infection cushion formation [GO:0075184]; positively regulated by positive regulation of infection cushion formation [GO:0075185]; negatively regulated by negative regulation of infection cushion formation [GO:0075186]